ABC-type glycerol-3-phosphate transporter activity [GO:0015430] (MF) Sources: RHEA:21668 Definition: Enables the transfer of a solute or solutes from one side of a membrane to the other according to the reaction: ATP + H2O + glycerol-3-phosphate(out) = ADP + phosphate + glycerol-3-phosphate(in). Also known as: ABC-type glycerol 3-phosphate transporter, glycerol-3-phosphate ABC transporter, ATP-dependent glycerol-2-phosphate transmembrane transporter activity, ATPase-coupled glycerol-2-phosphate transmembrane transporter activity, glycerol phosphate-importing ATPase activity, glycerol-2-phosphate-transporting ATPase activity, glycerol-phosphate porter activity, ATPase-coupled glycerol-3-phosphate transmembrane transporter activity, glycerol-3-phosphate-transporting ATPase Relationships: is a type of glycerol-3-phosphate transmembrane transporter activity [GO:0015169]; is a type of GO:0140359